nonfunctional rRNA decay [GO:0070651] (biological process) Relationships: is a type of rRNA catabolic process [GO:0016075] References: PMID:17188037, PMID:19390089 Sources: GOC:mah, GOC:rn Also known as: NRD Definition: An rRNA catabolic process that results in the targeted detection and degradation of aberrant rRNAs contained within translationally defective ribosomes, thereby acting as a quality-control system.